response to molecule of fungal origin [GO:0002238] (biological process) Relationships: is_a response to external biotic stimulus [GO:0043207]; is part of response to fungus [GO:0009620] Subtypes: detection of molecule of fungal origin [GO:0032491], cellular response to molecule of fungal origin [GO:0071226] Definition: Any process that results in a change in state or activity of an organism (in terms of movement, secretion, enzyme production, gene expression, etc.) as a result of a stimulus by molecules of fungal origin such as chito-octamer oligosaccharide. Sources: GOC:rl, GOC:sm Also known as: response to fungus associated molecule